{
  "gene": "UniProtKB:O95473",
  "gene_name": "Synaptogyrin-4",
  "term_label": "Unknown biological process",
  "term_id": "UNKNOWN:0002",
  "gene_symbol": "SYNGR4"
}